mesonephros development [GO:0001823] (biological process) Relationships: is a type of GO:0001822 Also known as: Wolffian body development References: PMID:10535314 Sources: GOC:dph, ISBN:0124020607, ISBN:0721662544 Definition: The process whose specific outcome is the progression of the mesonephros over time, from its formation to the mature structure. In mammals, the mesonephros is the second of the three embryonic kidneys to be established and exists only transiently. In lower vertebrates such as fish and amphibia, the mesonephros will form the mature kidney. Regulation: positively regulated by GO:0061213; regulated by regulation of mesonephros development [GO:0061217]; negatively regulated by negative regulation of mesonephros development [GO:0061218]